{
  "gene": "UniProtKB:P0DMU9",
  "gene_symbol": "CT45A10",
  "term_id": "UNKNOWN:0001",
  "gene_name": "Cancer_testis antigen family 45 member A10",
  "term_label": "Unknown molecular function"
}